{
  "term_id": "GO:0005615",
  "gene": "UniProtKB:P05452",
  "gene_symbol": "CLEC3B",
  "term_label": "extracellular space",
  "gene_name": "Tetranectin"
}